{
  "term_id": "GO:0000149",
  "gene_symbol": "STX5",
  "term_label": "SNARE binding",
  "gene": "UniProtKB:Q13190",
  "gene_name": "Syntaxin-5"
}